pentacyclic triterpenoid catabolic process [GO:0019741] (biological process) Sources: ISBN:0198506732 Subtypes: GO:1902382, glycyrrhetinate catabolic process [GO:1902385] Definition: The chemical reactions and pathways resulting in the breakdown of pentacyclic triterpenoid compounds, terpenoids with six isoprene units and 5 carbon rings. Also known as: pentacyclic triterpenoid breakdown, pentacyclic triterpenoid catabolism, pentacyclic triterpenoid degradation Relationships: is a type of triterpenoid catabolic process [GO:0016105]; is_a pentacyclic triterpenoid metabolic process [GO:0019742]